{
  "term_id": "GO:0016236",
  "gene": "UniProtKB:P49754",
  "gene_name": "Vacuolar protein sorting-associated protein 41 homolog",
  "term_label": "macroautophagy",
  "gene_symbol": "VPS41"
}